{
  "term_label": "cytoskeleton",
  "gene_symbol": "DYRK2",
  "gene_name": "Dual specificity tyrosine-phosphorylation-regulated kinase 2",
  "term_id": "GO:0005856",
  "gene": "UniProtKB:Q92630"
}